{
  "term_label": "Unknown molecular function",
  "gene": "UniProtKB:P57678",
  "gene_symbol": "GEMIN4",
  "term_id": "UNKNOWN:0001",
  "gene_name": "Gem-associated protein 4"
}